{
  "gene_name": "AMMECR1-like protein",
  "term_label": "Unknown molecular function",
  "term_id": "UNKNOWN:0001",
  "gene": "UniProtKB:Q6DCA0",
  "gene_symbol": "AMMECR1L"
}